{
  "gene": "UniProtKB:Q5FYB1",
  "term_label": "Unknown biological process",
  "gene_name": "Arylsulfatase I",
  "gene_symbol": "ARSI",
  "term_id": "UNKNOWN:0002"
}